{
  "term_id": "GO:0005743",
  "gene_symbol": "SFXN3",
  "gene": "UniProtKB:Q9BWM7",
  "term_label": "mitochondrial inner membrane",
  "gene_name": "Sideroflexin-3"
}